{
  "gene_name": "Poly(A)-specific ribonuclease PNLDC1",
  "term_label": "3'-5'-RNA exonuclease activity",
  "term_id": "GO:0000175",
  "gene": "UniProtKB:Q8NA58",
  "gene_symbol": "PNLDC1"
}